{
  "gene_symbol": "MCM3AP",
  "gene": "UniProtKB:O60318",
  "term_label": "mRNA export from nucleus",
  "term_id": "GO:0006406",
  "gene_name": "Germinal-center associated nuclear protein"
}